{
  "gene_name": "Keratin, type I cuticular Ha2",
  "term_label": "intermediate filament organization",
  "gene": "UniProtKB:Q14532",
  "term_id": "GO:0045109",
  "gene_symbol": "KRT32"
}